microvesicle [GO:1990742] (cellular component) Subtypes: GO:0098875 Relationships: is a type of extracellular vesicle [GO:1903561] Also known as: shedding vesicle, ectosome, extracellular microvesicle Definition: An extracellular vesicle released from the plasma membrane and ranging in size from about 100 nm to 1000 nm. References: PMID:22418571, PMID:24009894 Sources: GOC:vesicles, Wikipedia:Microvesicles